{
  "term_id": "GO:0003714",
  "gene": "UniProtKB:Q9UKL0",
  "gene_name": "REST corepressor 1",
  "gene_symbol": "RCOR1",
  "term_label": "transcription corepressor activity"
}